{
  "gene_symbol": "GAGE4",
  "gene": "UniProtKB:P0DSO3",
  "gene_name": "G antigen 4",
  "term_id": "UNKNOWN:0001",
  "term_label": "Unknown molecular function"
}